{
  "term_label": "Unknown molecular function",
  "gene": "UniProtKB:A8MYV0",
  "gene_name": "Doublecortin domain-containing protein 2C",
  "term_id": "UNKNOWN:0001",
  "gene_symbol": "DCDC2C"
}